{
  "gene_symbol": "CCDC196",
  "term_label": "Unknown cellular component",
  "gene": "UniProtKB:A0A1B0GTZ2",
  "term_id": "UNKNOWN:0003",
  "gene_name": "Putative coiled-coil domain-containing protein 196"
}